programmed cell death involved in cell development [GO:0010623] (biological process) Sources: GOC:dph, GOC:mtg_apoptosis, GOC:tb Subtypes: central B cell deletion [GO:0002342], synergid death [GO:0010198], larval midgut cell programmed cell death [GO:0035096], ectopic germ cell programmed cell death [GO:0035234], GO:0045476, retinal cell programmed cell death [GO:0046666], antipodal cell degeneration [GO:0055045] Definition: The activation of endogenous cellular processes that result in the death of a cell as part of its development. Relationships: is a type of programmed cell death [GO:0012501]; is a type of cellular developmental process [GO:0048869]; is part of GO:0048468 Note: This process is part of the natural developmental program of some cell types, but it does not always happen as part of the development or shaping of a gross anatomical structure. Also known as: developmental programmed cell death, programmed cell death involved in development